{
  "gene_symbol": "ITGA2B",
  "term_label": "cell-cell adhesion",
  "term_id": "GO:0098609",
  "gene": "UniProtKB:P08514",
  "gene_name": "Integrin alpha-IIb"
}